{
  "gene_name": "Carboxy-terminal domain RNA polymerase II polypeptide A small phosphatase 1",
  "term_label": "RNA polymerase II CTD heptapeptide repeat phosphatase activity",
  "gene": "UniProtKB:Q9GZU7",
  "term_id": "GO:0008420",
  "gene_symbol": "CTDSP1"
}